protein-phytochromobilin linkage [GO:0017012] (biological process) Sources: RESID:AA0133 Relationships: is a type of protein-bilin linkage [GO:0017007] Definition: The linkage of the chromophore phytochromobilin to phycocyanin or allophycocyanin.